{
  "gene": "UniProtKB:Q00G26",
  "term_label": "lipid storage",
  "term_id": "GO:0019915",
  "gene_symbol": "PLIN5",
  "gene_name": "Perilipin-5"
}